{
  "term_label": "Unknown molecular function",
  "gene_symbol": "NCDN",
  "gene": "UniProtKB:Q9UBB6",
  "term_id": "UNKNOWN:0001",
  "gene_name": "Neurochondrin"
}